{
  "gene_name": "Calpain-7",
  "gene_symbol": "CAPN7",
  "term_label": "cysteine-type endopeptidase activity",
  "term_id": "GO:0004197",
  "gene": "UniProtKB:Q9Y6W3"
}